regulation of intestinal epithelial structure maintenance [GO:0060730] (biological process) Sources: GOC:BHF, GOC:dph, GOC:tb Definition: Any process that modulates the rate, frequency, or extent of intestinal epithelial structure maintenance, a tissue homeostatic process required for the maintenance of the structure of the intestinal epithelium. Relationships: is a type of regulation of digestive system process [GO:0044058]; regulates intestinal epithelial structure maintenance [GO:0060729] Subtypes: positive regulation of intestinal epithelial structure maintenance [GO:0060731]